{
  "gene_symbol": "APRT",
  "term_label": "adenine binding",
  "gene": "UniProtKB:P07741",
  "gene_name": "Adenine phosphoribosyltransferase",
  "term_id": "GO:0002055"
}